{
  "term_label": "adaptive immune response",
  "gene_symbol": "IFNA21",
  "term_id": "GO:0002250",
  "gene_name": "Interferon alpha-21",
  "gene": "UniProtKB:P01568"
}